{
  "term_id": "GO:0042826",
  "gene": "UniProtKB:Q06413",
  "term_label": "histone deacetylase binding",
  "gene_name": "Myocyte-specific enhancer factor 2C",
  "gene_symbol": "MEF2C"
}